{
  "gene_name": "Interleukin-1 receptor-associated kinase 1",
  "term_id": "GO:0045087",
  "gene": "UniProtKB:P51617",
  "term_label": "innate immune response",
  "gene_symbol": "IRAK1"
}